{
  "gene": "UniProtKB:O15205",
  "term_label": "nucleus",
  "gene_name": "Ubiquitin D",
  "gene_symbol": "UBD",
  "term_id": "GO:0005634"
}